{
  "gene_name": "Transmembrane protein 14EP",
  "term_label": "heme biosynthetic process",
  "gene": "UniProtKB:Q6UXP3",
  "term_id": "GO:0006783",
  "gene_symbol": "TMEM14EP"
}